{
  "term_label": "nucleus",
  "term_id": "GO:0005634",
  "gene_name": "Postacrosomal sheath WW domain-binding protein",
  "gene_symbol": "WBP2NL",
  "gene": "UniProtKB:Q6ICG8"
}